all-trans retinal 3,4-desaturase activity [GO:0061897] (molecular function) References: PMID:27059013 Relationships: is a type of oxidoreductase activity, acting on paired donors, with incorporation or reduction of molecular oxygen [GO:0016705] Definition: Catalysis of the reaction: all-trans-retinal + 2 H+ + O2 + 2 reduced [adrenodoxin] = all-trans-3,4-didehydro retinal + 2 H2O + 2 oxidized [adrenodoxin].